S-sulfolactate dehydrogenase activity [GO:0102155] (molecular function) Definition: Catalysis of the reaction: (S)-3-sulfonatolactate + NAD = 3-sulfonatopyruvate(2-) + NADH + H+. Sources: EC:1.1.1.310, GOC:pz Relationships: is_a oxidoreductase activity, acting on the CH-OH group of donors, NAD or NADP as acceptor [GO:0016616]